methylammonium transmembrane transporter activity [GO:0015200] (molecular function) Definition: Enables directed movement of methylammonium, CH3NH2, from one side of a membrane to the other. Sources: GOC:ai Relationships: is a type of amine transmembrane transporter activity [GO:0005275]; BFO_0000050 methylammonium transmembrane transport [GO:0072489] Subtypes: GO:0015264